{
  "gene_symbol": "NPR2",
  "term_label": "natriuretic peptide receptor activity",
  "term_id": "GO:0016941",
  "gene_name": "Atrial natriuretic peptide receptor 2",
  "gene": "UniProtKB:P20594"
}